{
  "term_id": "GO:0050839",
  "term_label": "cell adhesion molecule binding",
  "gene_symbol": "PCDHGA7",
  "gene": "UniProtKB:Q9Y5G6",
  "gene_name": "Protocadherin gamma-A7"
}